lysine:cadaverine antiporter activity [GO:0043872] (molecular function) References: PMID:10986235 Sources: GOC:jl, TC:2.A.3.2.2 Also known as: cadaverine:lysine antiporter activity, lysine-cadaverine antiporter activity, lysine/cadaverine antiporter activity, cadaverine transmembrane transporter activity Relationships: is a type of amino acid transmembrane transporter activity [GO:0015171]; is a type of antiporter activity [GO:0015297]; is a type of GO:0046943 Definition: Catalysis of the reaction: lysine(out) + cadaverine(in) = lysine(in) + cadaverine(out).